tRNA (guanosine(34)-2'-O)-methyltransferase activity [GO:0106340] (molecular function) References: PMID:31943105 Definition: Catalysis of the reaction: guanosine(34) in tRNA + S-adenosyl-L-methionine = 2'-O-methylguanosine(34) in tRNA + H+ + S-adenosyl-L-homocysteine. Relationships: is_a GO:0016423